{
  "term_label": "mRNA binding",
  "gene_symbol": "CNBP",
  "gene_name": "CCHC-type zinc finger nucleic acid binding protein",
  "term_id": "GO:0003729",
  "gene": "UniProtKB:P62633"
}